{
  "term_id": "GO:0000027",
  "gene_name": "Midasin",
  "term_label": "ribosomal large subunit assembly",
  "gene": "UniProtKB:Q9NU22",
  "gene_symbol": "MDN1"
}